{
  "gene_name": "E3 ubiquitin-protein ligase CHFR",
  "gene": "UniProtKB:Q96EP1",
  "gene_symbol": "CHFR",
  "term_id": "GO:0004842",
  "term_label": "ubiquitin-protein transferase activity"
}